positive regulation of multicellular organism growth [GO:0040018] (BP) Definition: Any process that activates or increases the frequency, rate or extent of growth of an organism to reach its usual body size. Sources: GOC:dph, GOC:go_curators, GOC:tb Also known as: positive regulation of body growth, positive regulation of body size Relationships: is a type of GO:0040014; is a type of positive regulation of developmental growth [GO:0048639]; is a type of positive regulation of multicellular organismal process [GO:0051240]; positively regulates GO:0035264